choline transmembrane transporter activity [GO:0015220] (MF) Relationships: is_a transmembrane transporter activity [GO:0022857]; is part of choline transport [GO:0015871] Subtypes: choline:sodium symporter activity [GO:0005307], ABC-type choline transporter activity [GO:0033266] Definition: Enables the transfer of choline from one side of a membrane to the other. Choline (2-hydroxyethyltrimethylammonium) is an amino alcohol that occurs widely in living organisms as a constituent of certain types of phospholipids and in the neurotransmitter acetylcholine. Also known as: choline permease activity, amino acid/choline transmembrane transporter activity Sources: GOC:ai